positive regulation of autophagic cell death [GO:1904094] (biological process) Relationships: is a type of positive regulation of programmed cell death [GO:0043068]; is_a regulation of autophagic cell death [GO:1904092]; positively regulates GO:0048102 Definition: Any process that activates or increases the frequency, rate or extent of autophagic cell death. Also known as: positive regulation of programmed cell death by macroautophagy, up regulation of autophagic cell death, up regulation of programmed cell death by macroautophagy, up-regulation of autophagic cell death, up-regulation of programmed cell death by macroautophagy, upregulation of autophagic cell death, upregulation of programmed cell death by macroautophagy, activation of autophagic cell death, activation of programmed cell death by macroautophagy, activation of type II programmed cell death, positive regulation of type II programmed cell death, up regulation of type II programmed cell death, up-regulation of type II programmed cell death, upregulation of type II programmed cell death References: PMID:25736836 Sources: GOC:TermGenie, GOC:bhm, GO_REF:0000058